diphosphoinositol polyphosphate metabolic process [GO:0071543] (biological process) Subtypes: diphosphoinositol polyphosphate catabolic process [GO:0071544] Relationships: is a type of GO:0043647 Definition: The chemical reactions and pathways involving a diphosphoinositol polyphosphate, 1,2,3,4,5,6-cyclohexanehexol with one or more diphosphate groups and multiple monophosphate groups attached. Also known as: diphosphoinositol polyphosphate metabolism References: PMID:12387729 Sources: GOC:mah